{
  "gene_name": "DnaJ homolog subfamily C member 3",
  "gene_symbol": "DNAJC3",
  "term_id": "GO:0005783",
  "gene": "UniProtKB:Q13217",
  "term_label": "endoplasmic reticulum"
}